cis-1,2-dihydro-1,2-dihydroxynaphthalene dehydrogenase activity [GO:0018505] (molecular function) Relationships: is a type of oxidoreductase activity, acting on the CH-CH group of donors, NAD or NADP as acceptor [GO:0016628] Definition: Catalysis of the reaction: cis-1,2-dihydronaphthalene-1,2-diol + NAD+ = naphthalene-1,2-diol + NADH + H+. Also known as: 1,2-dihydroxy-1,2-dihydroxynaphthalene dehydrogenase activity, (+)-cis-naphthalene dihydrodiol dehydrogenase activity, cis-1,2-dihydronaphthalene-1,2-diol:NAD+ 1,2-oxidoreductase activity, cis-dihydrodiol naphthalene dehydrogenase activity, cis-naphthalene dihydrodiol dehydrogenase activity, naphthalene dihydrodiol dehydrogenase activity Sources: EC:1.3.1.29